{
  "term_id": "GO:0007165",
  "gene_name": "Rho-related GTP-binding protein RhoC",
  "gene": "UniProtKB:P08134",
  "gene_symbol": "RHOC",
  "term_label": "signal transduction"
}